indole-3-acetaldehyde reductase (NADH) activity [GO:0047018] (molecular function) Relationships: is a type of alcohol dehydrogenase (NAD+) activity [GO:0004022] Sources: EC:1.1.1.190, RHEA:14873 Definition: Catalysis of the reaction: indole-3-ethanol + NAD+ = (indol-3-yl)acetaldehyde + H+ + NADH. Also known as: (indol-3-yl)ethanol:NAD+ oxidoreductase activity, indole-3-ethanol:NAD+ oxidoreductase activity, indoleacetaldehyde reductase activity